dihydroorotate dehydrogenase activity [GO:0004152] (molecular function) Definition: Catalysis of the reaction: (S)-dihydroorotate + A = AH(2) + orotate. Sources: RHEA:18073 Relationships: is a type of oxidoreductase activity, acting on the CH-CH group of donors [GO:0016627] Subtypes: dihydroorotate dehydrogenase (NAD+) activity [GO:0004589], GO:0050158, GO:0106430, GO:1990663